{
  "term_id": "UNKNOWN:0002",
  "term_label": "Unknown biological process",
  "gene": "UniProtKB:Q8N8A2",
  "gene_symbol": "ANKRD44",
  "gene_name": "Serine_threonine-protein phosphatase 6 regulatory ankyrin repeat subunit B"
}